alphav-beta3 integrin-ADAM15 complex [GO:0071057] (cellular component) Definition: A protein complex that consists of an alphav-beta3 integrin complex bound to the transmembrane metallopeptidase ADAM15. References: PMID:10944520, PMID:11882657 Also known as: ITGAV-ITGB3-ADAM15 complex Relationships: is a type of plasma membrane protein complex [GO:0098797]; is a type of catalytic complex [GO:1902494]